{
  "gene": "UniProtKB:Q86YL7",
  "term_label": "basolateral plasma membrane",
  "gene_symbol": "PDPN",
  "gene_name": "Podoplanin",
  "term_id": "GO:0016323"
}